{
  "gene_symbol": "DIS3L2",
  "term_id": "GO:0000932",
  "gene_name": "DIS3-like exonuclease 2",
  "gene": "UniProtKB:Q8IYB7",
  "term_label": "P-body"
}